peptide 2-hydroxyisobutyryltransferase activity [GO:0106226] (molecular function) References: PMID:29775581 Sources: GOC:sp Definition: Catalysis of the reaction: 2-hydroxyisobutyryl-CoA + lysine in peptide = CoA + N-2-hydroxyisobutyryl-lysine-peptide. Relationships: is a type of N-acyltransferase activity [GO:0016410]